{
  "gene": "UniProtKB:Q9UJX6",
  "gene_name": "Anaphase-promoting complex subunit 2",
  "term_id": "GO:0005680",
  "term_label": "anaphase-promoting complex",
  "gene_symbol": "ANAPC2"
}